{
  "gene_name": "Abl interactor 2",
  "term_label": "neuron migration",
  "gene": "UniProtKB:Q9NYB9",
  "term_id": "GO:0001764",
  "gene_symbol": "ABI2"
}